{
  "gene_symbol": "MMP12",
  "gene_name": "Macrophage metalloelastase",
  "gene": "UniProtKB:P39900",
  "term_id": "GO:0030574",
  "term_label": "collagen catabolic process"
}